{
  "gene": "UniProtKB:Q06830",
  "term_label": "cytosol",
  "term_id": "GO:0005829",
  "gene_symbol": "PRDX1",
  "gene_name": "Peroxiredoxin-1"
}